{
  "term_label": "glutathione hydrolase activity",
  "term_id": "GO:0036374",
  "gene": "UniProtKB:Q9UJ14",
  "gene_symbol": "GGT7",
  "gene_name": "Glutathione hydrolase 7"
}